{
  "term_id": "GO:0015269",
  "term_label": "calcium-activated potassium channel activity",
  "gene_symbol": "KCNMB1",
  "gene_name": "Calcium-activated potassium channel subunit beta-1",
  "gene": "UniProtKB:Q16558"
}